phosphatase binding [GO:0019902] (molecular function) Definition: Binding to a phosphatase. Sources: GOC:jl Relationships: is_a enzyme binding [GO:0019899] Subtypes: protein phosphatase binding [GO:0019903]